{
  "term_id": "GO:0031012",
  "gene_name": "Testican-3",
  "term_label": "extracellular matrix",
  "gene_symbol": "SPOCK3",
  "gene": "UniProtKB:Q9BQ16"
}